{
  "term_label": "estrogen response element binding",
  "gene_name": "Steroid hormone receptor ERR2",
  "term_id": "GO:0034056",
  "gene": "UniProtKB:O95718",
  "gene_symbol": "ESRRB"
}